positive regulation of raffinose biosynthetic process [GO:1900093] (biological process) Relationships: is a type of GO:0009891; is a type of positive regulation of carbohydrate metabolic process [GO:0045913]; is a type of regulation of raffinose biosynthetic process [GO:1900091]; positively regulates raffinose biosynthetic process [GO:0033529] Also known as: activation of raffinose anabolism, activation of raffinose biosynthesis, activation of raffinose formation, activation of raffinose synthesis, positive regulation of raffinose anabolism, positive regulation of raffinose biosynthesis, positive regulation of raffinose formation, positive regulation of raffinose synthesis, up regulation of raffinose anabolism, up regulation of raffinose biosynthesis, up regulation of raffinose biosynthetic process, up regulation of raffinose formation, up regulation of raffinose synthesis, up-regulation of raffinose anabolism, up-regulation of raffinose biosynthesis, up-regulation of raffinose biosynthetic process, up-regulation of raffinose formation, up-regulation of raffinose synthesis, upregulation of raffinose anabolism, upregulation of raffinose biosynthesis, upregulation of raffinose biosynthetic process, upregulation of raffinose formation, upregulation of raffinose synthesis, activation of raffinose biosynthetic process Definition: Any process that activates or increases the frequency, rate or extent of raffinose biosynthetic process. References: PMID:22307851 Sources: GOC:TermGenie